{
  "gene_name": "Dead end protein homolog 1",
  "term_id": "GO:0005634",
  "term_label": "nucleus",
  "gene_symbol": "DND1",
  "gene": "UniProtKB:Q8IYX4"
}